{
  "gene_symbol": "TRGV2",
  "gene_name": "T cell receptor gamma variable 2",
  "gene": "UniProtKB:A0A075B6R0",
  "term_label": "Unknown cellular component",
  "term_id": "UNKNOWN:0003"
}